epithelial cell proliferation involved in prostate gland development [GO:0060767] (biological process) Subtypes: GO:0060517 Definition: The multiplication or reproduction of epithelial cells, resulting in the expansion of a cell population that contributes to the progression of the prostate gland over time. Regulation: regulated by regulation of epithelial cell proliferation involved in prostate gland development [GO:0060768]; positively regulated by positive regulation of epithelial cell proliferation involved in prostate gland development [GO:0060769]; negatively regulated by negative regulation of epithelial cell proliferation involved in prostate gland development [GO:0060770] Sources: GOC:dph Relationships: is a type of epithelial cell proliferation [GO:0050673]; is part of prostate gland development [GO:0030850]